nylon catabolic process [GO:0019876] (biological process) Definition: The chemical reactions and pathways resulting in the breakdown of nylon, a polymer where the main polymer chain comprises recurring amide groups; these compounds are generally formed from combinations of diamines, diacids and amino acids. Sources: UniProtKB-KW:KW-0549 Also known as: nylon breakdown, nylon catabolism, nylon degradation Relationships: is a type of GO:0042178